{
  "gene": "UniProtKB:Q5JX71",
  "gene_name": "Protein FAM209A",
  "gene_symbol": "FAM209A",
  "term_id": "UNKNOWN:0003",
  "term_label": "Unknown cellular component"
}